{
  "term_id": "GO:0034334",
  "gene_symbol": "MTSS1",
  "gene": "UniProtKB:O43312",
  "term_label": "adherens junction maintenance",
  "gene_name": "Protein MTSS 1"
}